{
  "term_label": "bicellular tight junction",
  "gene_name": "Claudin-17",
  "gene": "UniProtKB:P56750",
  "gene_symbol": "CLDN17",
  "term_id": "GO:0005923"
}